{
  "gene": "UniProtKB:A8MTZ0",
  "term_id": "GO:0097500",
  "gene_symbol": "BBIP1",
  "gene_name": "BBSome-interacting protein 1",
  "term_label": "receptor localization to non-motile cilium"
}